polymeric IgA immunoglobulin complex [GO:0071749] (cellular component) Also known as: pIgA antibody, polymeric IgA antibody, pIgA1 antibody, polymeric IgA1 antibody Note: Note that an IgA immunoglobulin complex has the function of antigen binding if a suitable antigen is available. Dimeric IgA is by far the most common form of polymeric IgA. In human only the IgA1 isotype is capable of a polymeric forms. Relationships: is_a GO:0071746 Subtypes: dimeric IgA immunoglobulin complex [GO:0071750], secretory IgA immunoglobulin complex [GO:0071751] References: PMID:16362985 Sources: GOC:add, ISBN:0781765196 Definition: A protein complex composed of two, three, or four monomeric IgA immunoglobulin complexes linked through both direct disulfide bonds and through disulfide binded monomers of J chain acting as a bridge. Each IgA monomer consists of two identical immunoglobulin heavy chains of an IgA isotype and two identical immunoglobulin light chains, held together by disulfide bonds. Dimeric IgA is sometimes complexed additionally with secretory component, and present in the extracellular space, in mucosal areas or other tissues, or circulating in the blood or lymph.